positive regulation of vascular wound healing [GO:0035470] (biological process) Relationships: is a type of positive regulation of angiogenesis [GO:0045766]; is a type of regulation of vascular wound healing [GO:0061043]; is a type of positive regulation of wound healing [GO:0090303]; positively regulates vascular wound healing [GO:0061042] Sources: GOC:rph Definition: Any process that increases the rate, frequency, or extent of blood vessel formation when new vessels emerge from the proliferation of pre-existing blood vessels and contribute to the series of events that restore integrity to damaged vasculature.